dirigent protein activity [GO:0102910] (molecular function) References: PMID:37202648 Sources: GOC:pz, MetaCyc:RXN-8677 Relationships: is_a molecular_function [GO:0003674] Definition: Catalysis of the reaction: 2 H+ + 2 coniferol + O2 = (+)-pinoresinol + 2 H2O. The The protein encoding this activity has been termed 'dirigent protein' because it does not express any catalytic activity and serves only to bind and orientate the coniferyl alcohol-derived free radicals.